positive regulation of timing of catagen [GO:0051795] (biological process) Relationships: is a type of GO:0048818; is a type of regulation of timing of catagen [GO:0051794]; positively regulates catagen [GO:0042637] Definition: Any process that activates or increases the frequency, rate or extent of timing of catagen, the regression phase of the hair cycle. Sources: GOC:ai, GOC:pr Also known as: activation of catagen, stimulation of catagen, positive regulation of catagen, up regulation of catagen, up-regulation of catagen, upregulation of catagen